{
  "term_id": "UNKNOWN:0001",
  "gene_name": "Sperm protein associated with the nucleus on the X chromosome N2",
  "gene": "UniProtKB:Q5MJ10",
  "gene_symbol": "SPANXN2",
  "term_label": "Unknown molecular function"
}